intermediate mesodermal cell fate commitment [GO:0048393] (biological process) Relationships: is a type of mesodermal cell fate commitment [GO:0001710]; is part of intermediate mesodermal cell differentiation [GO:0048392] Definition: The process in which the developmental fate of a cell becomes restricted such that it will develop into an intermediate mesoderm cell. Sources: GOC:dgh Also known as: intermediate mesoderm cell fate commitment